{
  "gene_name": "Dehydrogenase_reductase SDR family member 4",
  "gene_symbol": "DHRS4",
  "term_label": "retinal metabolic process",
  "term_id": "GO:0042574",
  "gene": "UniProtKB:Q9BTZ2"
}